{
  "gene_symbol": "KATNA1",
  "term_label": "cytoplasm",
  "term_id": "GO:0005737",
  "gene": "UniProtKB:O75449",
  "gene_name": "Katanin p60 ATPase-containing subunit A1"
}